{
  "term_id": "UNKNOWN:0002",
  "gene": "UniProtKB:B3KNS4",
  "term_label": "Unknown biological process",
  "gene_name": "Endogenous retrovirus group K3 member 1",
  "gene_symbol": "ERVK3-1"
}